{
  "gene_symbol": "VIP",
  "term_label": "regulation of protein localization",
  "gene_name": "VIP peptides",
  "term_id": "GO:0032880",
  "gene": "UniProtKB:P01282"
}